{
  "term_id": "GO:0045087",
  "gene_symbol": "TRIM22",
  "term_label": "innate immune response",
  "gene": "UniProtKB:Q8IYM9",
  "gene_name": "E3 ubiquitin-protein ligase TRIM22"
}